endothelial cell activation involved in immune response [GO:0002264] (biological process) Relationships: is a type of cell activation involved in immune response [GO:0002263]; is a type of endothelial cell activation [GO:0042118] Also known as: endothelial cell activation during immune response Definition: A change in the morphology or behavior of an endothelial cell resulting from exposure to an activating factor such as a cellular or soluble ligand, leading to the initiation or perpetuation of an immune response. Sources: GOC:add, ISBN:0781735149 Subtypes: endothelial cell activation within high endothelial venule involved in immune response [GO:0002259]